{
  "term_label": "Unknown biological process",
  "term_id": "UNKNOWN:0002",
  "gene_name": "OCIA domain-containing protein 2",
  "gene": "UniProtKB:Q56VL3",
  "gene_symbol": "OCIAD2"
}